{
  "gene_symbol": "GRAPL",
  "gene_name": "GRB2-related adapter protein-like",
  "term_id": "GO:0016477",
  "gene": "UniProtKB:Q8TC17",
  "term_label": "cell migration"
}